{
  "gene_name": "Partitioning defective 3 homolog",
  "gene_symbol": "PARD3",
  "term_label": "microtubule cytoskeleton organization",
  "term_id": "GO:0000226",
  "gene": "UniProtKB:Q8TEW0"
}